regulation of epithelial cell migration, open tracheal system [GO:2000274] (biological process) Also known as: regulation of tracheal cell migration, regulation of tracheal epithelial cell migration Definition: Any process that modulates the frequency, rate or extent of epithelial cell migration, open tracheal system. Relationships: is a type of regulation of epithelial cell migration [GO:0010632]; regulates epithelial cell migration, open tracheal system [GO:0007427] Sources: GOC:obol